{
  "gene_name": "Serine_threonine-protein phosphatase 4 regulatory subunit 3B",
  "term_label": "protein phosphatase 4 complex",
  "gene_symbol": "PPP4R3B",
  "term_id": "GO:0030289",
  "gene": "UniProtKB:Q5MIZ7"
}